{
  "term_label": "regulation of transcription by RNA polymerase II",
  "gene": "UniProtKB:O95696",
  "gene_symbol": "BRD1",
  "gene_name": "Bromodomain-containing protein 1",
  "term_id": "GO:0006357"
}